{
  "term_label": "nucleus",
  "gene_symbol": "TSPY1",
  "gene": "UniProtKB:Q01534",
  "gene_name": "Testis-specific Y-encoded protein 1",
  "term_id": "GO:0005634"
}